ribonucleoside-triphosphate reductase (thioredoxin) activity [GO:0008998] (molecular function) Sources: RHEA:12701 Relationships: is a type of oxidoreductase activity, acting on CH or CH2 groups, disulfide as acceptor [GO:0016728] Also known as: ribonucleotide reductase activity, ribonucleoside-triphosphate reductase activity, 2'-deoxyribonucleoside-triphosphate:oxidized-thioredoxin 2'-oxidoreductase activity, 2'-deoxyribonucleoside-triphosphate:thioredoxin-disulfide 2'-oxidoreductase activity Definition: Catalysis of the reaction: [thioredoxin]-disulfide + a 2'-deoxyribonucleoside 5'-triphosphate + H2O = [thioredoxin]-dithiol + a ribonucleoside 5'-triphosphate.